{
  "gene": "UniProtKB:Q9UPR5",
  "term_label": "sarcolemma",
  "gene_name": "Sodium_calcium exchanger 2",
  "term_id": "GO:0042383",
  "gene_symbol": "SLC8A2"
}